{
  "gene_symbol": "EMC9",
  "gene": "UniProtKB:Q9Y3B6",
  "term_label": "protein insertion into ER membrane by stop-transfer membrane-anchor sequence",
  "term_id": "GO:0045050",
  "gene_name": "ER membrane protein complex subunit 9"
}